L-erythro-3,5-diaminohexanoate dehydrogenase activity [GO:0047124] (molecular function) Definition: Catalysis of the reaction: (3S,5S)-3,5-diaminohexanoate + H2O + NAD+ = (S)-5-amino-3-oxo-hexanoate + H+ + NADH + NH4. Sources: EC:1.4.1.11, RHEA:19633 Relationships: is a type of oxidoreductase activity, acting on the CH-NH2 group of donors, NAD or NADP as acceptor [GO:0016639] Also known as: L-3,5-diaminohexanoate dehydrogenase activity, L-erythro-3,5-diaminohexanoate:NAD+ oxidoreductase (deaminating)